{
  "term_id": "GO:0120020",
  "gene": "UniProtKB:P02649",
  "gene_name": "Apolipoprotein E",
  "gene_symbol": "APOE",
  "term_label": "cholesterol transfer activity"
}